{
  "gene_name": "Peroxisome proliferator-activated receptor gamma coactivator 1-beta",
  "gene_symbol": "PPARGC1B",
  "gene": "UniProtKB:Q86YN6",
  "term_label": "nucleus",
  "term_id": "GO:0005634"
}